protein localization to trailing edge [GO:0036051] (biological process) Relationships: is a type of intracellular protein localization [GO:0008104] Subtypes: GO:0036052 Sources: GOC:pf, GOC:pg Also known as: protein localisation to trailing edge Definition: A process in which a protein is transported to, or maintained at, the trailing edge. The trailing edge is the area of a motile cell opposite to the direction of movement.